{
  "term_label": "immune response",
  "term_id": "GO:0006955",
  "gene_name": "Interleukin-1 family member 10",
  "gene": "UniProtKB:Q8WWZ1",
  "gene_symbol": "IL1F10"
}